{
  "gene_name": "Kelch-like protein 25",
  "gene_symbol": "KLHL25",
  "term_label": "Cul3-RING ubiquitin ligase complex",
  "term_id": "GO:0031463",
  "gene": "UniProtKB:Q9H0H3"
}